{
  "gene": "UniProtKB:Q6ZNA4",
  "gene_name": "E3 ubiquitin-protein ligase Arkadia",
  "gene_symbol": "RNF111",
  "term_id": "GO:0061630",
  "term_label": "ubiquitin protein ligase activity"
}